{
  "term_id": "GO:0005886",
  "gene_name": "FYN-binding protein 2",
  "term_label": "plasma membrane",
  "gene_symbol": "FYB2",
  "gene": "UniProtKB:Q5VWT5"
}